{
  "gene_name": "Putative malate dehydrogenase 1B",
  "term_id": "GO:0006099",
  "gene_symbol": "MDH1B",
  "gene": "UniProtKB:Q5I0G3",
  "term_label": "tricarboxylic acid cycle"
}